{
  "gene_symbol": "CLCN7",
  "term_id": "GO:0005765",
  "gene": "UniProtKB:P51798",
  "gene_name": "H(+)_Cl(-) exchange transporter 7",
  "term_label": "lysosomal membrane"
}